{
  "gene_name": "Sialidase-3",
  "gene": "UniProtKB:Q9UQ49",
  "gene_symbol": "NEU3",
  "term_id": "GO:0005737",
  "term_label": "cytoplasm"
}